{
  "gene": "UniProtKB:Q9H2X6",
  "term_label": "cytoplasm",
  "gene_name": "Homeodomain-interacting protein kinase 2",
  "gene_symbol": "HIPK2",
  "term_id": "GO:0005737"
}